{
  "term_id": "GO:0005871",
  "gene_symbol": "KIF17",
  "gene_name": "Kinesin-like protein KIF17",
  "gene": "UniProtKB:Q9P2E2",
  "term_label": "kinesin complex"
}